{
  "gene_name": "Calreticulin",
  "term_id": "GO:0006457",
  "term_label": "protein folding",
  "gene_symbol": "CALR",
  "gene": "UniProtKB:P27797"
}